{
  "gene": "UniProtKB:Q7Z5J1",
  "term_label": "Unknown biological process",
  "term_id": "UNKNOWN:0002",
  "gene_name": "Hydroxysteroid 11-beta-dehydrogenase 1-like protein",
  "gene_symbol": "HSD11B1L"
}